{
  "term_label": "beta-catenin binding",
  "term_id": "GO:0008013",
  "gene": "UniProtKB:Q9UI47",
  "gene_symbol": "CTNNA3",
  "gene_name": "Catenin alpha-3"
}